{
  "gene_name": "Otoconin-90",
  "gene_symbol": "OC90",
  "term_id": "GO:0005509",
  "gene": "UniProtKB:Q02509",
  "term_label": "calcium ion binding"
}